{
  "gene_symbol": "XCR1",
  "gene": "UniProtKB:P46094",
  "term_id": "GO:0006955",
  "term_label": "immune response",
  "gene_name": "Chemokine XC receptor 1"
}